{
  "term_label": "Unknown molecular function",
  "gene_symbol": "TMEM60",
  "term_id": "UNKNOWN:0001",
  "gene_name": "Transmembrane protein 60",
  "gene": "UniProtKB:Q9H2L4"
}